hyaluronic acid binding [GO:0005540] (molecular function) Sources: GOC:jl Definition: Binding to hyaluronic acid, a polymer composed of repeating dimeric units of glucuronic acid and N-acetyl glucosamine. Also known as: hyaluronan binding Relationships: is a type of glycosaminoglycan binding [GO:0005539]